{
  "gene_name": "Leucine-rich repeat-containing protein 37A",
  "term_id": "UNKNOWN:0001",
  "gene_symbol": "LRRC37A",
  "gene": "UniProtKB:A6NMS7",
  "term_label": "Unknown molecular function"
}